{
  "gene": "UniProtKB:Q8NFP7",
  "term_id": "GO:0005737",
  "term_label": "cytoplasm",
  "gene_name": "Diphosphoinositol polyphosphate phosphohydrolase 3-alpha",
  "gene_symbol": "NUDT10"
}